{
  "gene_symbol": "PPP1CC",
  "gene_name": "Serine_threonine-protein phosphatase PP1-gamma catalytic subunit",
  "term_id": "GO:0004722",
  "gene": "UniProtKB:P36873",
  "term_label": "protein serine/threonine phosphatase activity"
}